response to growth factor [GO:0070848] (biological process) Definition: Any process that results in a change in state or activity of a cell or an organism (in terms of movement, secretion, enzyme production, gene expression, etc.) as a result of a growth factor stimulus. Sources: GOC:BHF, GOC:mah Also known as: response to growth factor stimulus Relationships: is a type of GO:0009719 Subtypes: response to hepatocyte growth factor [GO:0035728], response to platelet-derived growth factor [GO:0036119], response to epidermal growth factor [GO:0070849], cellular response to growth factor stimulus [GO:0071363], response to transforming growth factor beta [GO:0071559], response to BMP [GO:0071772], response to fibroblast growth factor [GO:0071774], response to nerve growth factor [GO:1990089], GO:1990790